{
  "gene": "UniProtKB:Q9H6L5",
  "gene_symbol": "RETREG1",
  "term_id": "GO:0043524",
  "gene_name": "Reticulophagy regulator 1",
  "term_label": "negative regulation of neuron apoptotic process"
}